{
  "gene_name": "Bromodomain-containing protein 2",
  "term_id": "GO:0004674",
  "term_label": "protein serine/threonine kinase activity",
  "gene_symbol": "BRD2",
  "gene": "UniProtKB:P25440"
}